{
  "term_id": "GO:0005829",
  "gene_symbol": "ULK3",
  "term_label": "cytosol",
  "gene": "UniProtKB:Q6PHR2",
  "gene_name": "Serine_threonine-protein kinase ULK3"
}